{
  "term_id": "GO:0000978",
  "gene_name": "Zinc finger protein 784",
  "gene": "UniProtKB:Q8NCA9",
  "term_label": "RNA polymerase II cis-regulatory region sequence-specific DNA binding",
  "gene_symbol": "ZNF784"
}